{
  "gene_symbol": "CLXN",
  "gene_name": "Calaxin",
  "gene": "UniProtKB:Q9HAE3",
  "term_id": "GO:0009966",
  "term_label": "regulation of signal transduction"
}